polyamine binding [GO:0019808] (molecular function) Relationships: is a type of amine binding [GO:0043176] Sources: GOC:ai Definition: Binding to a polyamine, an organic compound containing two or more amino groups. Subtypes: spermidine binding [GO:0019809], GO:0019810